{
  "term_id": "UNKNOWN:0002",
  "gene": "UniProtKB:Q9Y324",
  "gene_symbol": "FCF1",
  "gene_name": "rRNA-processing protein FCF1 homolog",
  "term_label": "Unknown biological process"
}